{
  "gene": "UniProtKB:O14904",
  "term_label": "canonical Wnt signaling pathway",
  "gene_name": "Protein Wnt-9a",
  "gene_symbol": "WNT9A",
  "term_id": "GO:0060070"
}